{
  "term_label": "Unknown cellular component",
  "gene": "UniProtKB:Q92681",
  "gene_name": "Regulatory solute carrier protein family 1 member 1",
  "term_id": "UNKNOWN:0003",
  "gene_symbol": "RSC1A1"
}